{
  "gene": "UniProtKB:O95319",
  "term_label": "mRNA 3'-UTR binding",
  "gene_name": "CUGBP Elav-like family member 2",
  "gene_symbol": "CELF2",
  "term_id": "GO:0003730"
}